{
  "gene_name": "Biglycan",
  "gene_symbol": "BGN",
  "term_label": "extracellular space",
  "gene": "UniProtKB:P21810",
  "term_id": "GO:0005615"
}